{
  "term_id": "UNKNOWN:0002",
  "gene": "UniProtKB:Q6P1X6",
  "term_label": "Unknown biological process",
  "gene_symbol": "C8orf82",
  "gene_name": "UPF0598 protein C8orf82"
}